{
  "term_id": "UNKNOWN:0002",
  "gene_symbol": "FAHD2A",
  "gene": "UniProtKB:Q96GK7",
  "term_label": "Unknown biological process",
  "gene_name": "Fumarylacetoacetate hydrolase domain-containing protein 2A"
}